{
  "term_label": "immunoglobulin mediated immune response",
  "term_id": "GO:0016064",
  "gene": "UniProtKB:A0A0B4J1U7",
  "gene_symbol": "IGHV6-1",
  "gene_name": "Immunoglobulin heavy variable 6-1"
}